stomach fundus smooth muscle contraction [GO:0014825] (biological process) Definition: A process in which force is generated within smooth muscle tissue, resulting in a change in muscle geometry. This process occurs in the fundus of stomach. Force generation involves a chemo-mechanical energy conversion step that is carried out by the actin/myosin complex activity, which generates force through ATP hydrolysis. The fundus is the portion of the stomach that lies above the cardiac notch. Sources: GOC:mtg_muscle, MA:0001612 Relationships: is a type of proximal stomach smooth muscle contraction [GO:0014847] Regulation: regulated by regulation of stomach fundus smooth muscle contraction [GO:0120068]; positively regulated by positive regulation of stomach fundus smooth muscle contraction [GO:0120069]; negatively regulated by negative regulation of stomach fundus smooth muscle contraction [GO:0120070]